{
  "gene": "UniProtKB:Q92759",
  "term_label": "nucleotide-excision repair",
  "gene_symbol": "GTF2H4",
  "gene_name": "General transcription factor IIH subunit 4",
  "term_id": "GO:0006289"
}